Fc-epsilon receptor signaling pathway [GO:0038095] (biological process) Subtypes: GO:0038097 References: PMID:12413516, PMID:15048725 Sources: GOC:phg Definition: The series of molecular signals initiated by the binding of the Fc portion of immunoglobulin E (IgE) to an Fc-epsilon receptor on the surface of a target cell, and ending with the regulation of a downstream cellular process, e.g. transcription. The Fc portion of an immunoglobulin is its C-terminal constant region. Relationships: is a type of Fc receptor signaling pathway [GO:0038093] Also known as: Fc-epsilon receptor signalling pathway